{
  "gene_name": "Chromobox protein homolog 3",
  "gene_symbol": "CBX3",
  "gene": "UniProtKB:Q13185",
  "term_id": "GO:0005721",
  "term_label": "pericentric heterochromatin"
}